{
  "gene_name": "NLR family member X1",
  "gene": "UniProtKB:Q86UT6",
  "term_id": "GO:0039536",
  "gene_symbol": "NLRX1",
  "term_label": "negative regulation of RIG-I signaling pathway"
}